{
  "gene": "UniProtKB:P28161",
  "gene_name": "Glutathione S-transferase Mu 2",
  "term_id": "UNKNOWN:0003",
  "term_label": "Unknown cellular component",
  "gene_symbol": "GSTM2"
}